{
  "term_id": "GO:0030425",
  "gene": "UniProtKB:O43896",
  "term_label": "dendrite",
  "gene_name": "Kinesin-like protein KIF1C",
  "gene_symbol": "KIF1C"
}